{
  "term_label": "phosphatidylinositol dephosphorylation",
  "gene_symbol": "MTMR6",
  "gene": "UniProtKB:Q9Y217",
  "gene_name": "Myotubularin-related protein 6",
  "term_id": "GO:0046856"
}